{
  "term_label": "respiratory chain complex",
  "term_id": "GO:0098803",
  "gene": "UniProtKB:P24310",
  "gene_name": "Cytochrome c oxidase subunit 7A1, mitochondrial",
  "gene_symbol": "COX7A1"
}